Golgi cis cisterna [GO:0000137] (cellular component) Definition: The Golgi cisterna closest to the endoplasmic reticulum; the first processing compartment through which proteins pass after export from the ER. Relationships: is_a Golgi cisterna [GO:0031985] Sources: ISBN:0815316194 Also known as: Golgi apparatus cis cisterna